mitochondrial crista [GO:0030061] (cellular component) Sources: ISBN:0198506732 Relationships: is a type of GO:0110165; is part of mitochondrial inner membrane [GO:0005743] Definition: Any of the inward folds of the mitochondrial inner membrane. Their number, extent, and shape differ in mitochondria from different tissues and organisms. They appear to be devices for increasing the surface area of the mitochondrial inner membrane, where the enzymes of electron transport and oxidative phosphorylation are found. Their shape can vary with the respiratory state of the mitochondria. Note: See also the cellular component term 'mitochondrial inner membrane ; GO:0005743'. Also known as: cristae, mitochondrial cristae